{
  "gene_symbol": "VPS4B",
  "term_label": "ATP hydrolysis activity",
  "term_id": "GO:0016887",
  "gene": "UniProtKB:O75351",
  "gene_name": "Vacuolar protein sorting-associated protein 4B"
}